regulation of dopamine receptor signaling pathway [GO:0060159] (biological process) Sources: GOC:dph Also known as: regulation of dopamine receptor signalling pathway Relationships: is a type of GO:0008277; RO_0002211 G protein-coupled dopamine receptor signaling pathway [GO:0007212] Subtypes: GO:0060160, positive regulation of dopamine receptor signaling pathway [GO:0060161], regulation of adenylate cyclase-inhibiting dopamine receptor signaling pathway [GO:1904990] Definition: Any process that modulates the frequency, rate or extent of a dopamine receptor signaling pathway activity. A dopamine receptor signaling pathway is the series of molecular signals generated as a consequence of a dopamine receptor binding to one of its physiological ligands.